{
  "gene_name": "Putative protein ZNF321",
  "gene_symbol": "ZNF321P",
  "term_label": "Unknown cellular component",
  "gene": "UniProtKB:Q8N8H1",
  "term_id": "UNKNOWN:0003"
}